lupan-3beta,20-diol synthase activity [GO:0102245] (MF) Sources: EC:4.2.1.128, GOC:pz Relationships: is a type of hydro-lyase activity [GO:0016836] Definition: Catalysis of the reaction: lupan-3beta,20-diol = (S)-2,3-epoxysqualene + H2O.